negative regulation of interleukin-1-mediated signaling pathway [GO:2000660] (biological process) Sources: GOC:obol Relationships: is_a negative regulation of cytokine-mediated signaling pathway [GO:0001960]; is a type of regulation of interleukin-1-mediated signaling pathway [GO:2000659]; negatively regulates interleukin-1-mediated signaling pathway [GO:0070498] Also known as: negative regulation of IL-1-mediated signaling pathway, negative regulation of interleukin-1-mediated signalling pathway, negative regulation of IL-1 alpha-mediated signaling pathway, negative regulation of IL-1 beta-mediated signaling pathway, negative regulation of interleukin-1 alpha-mediated signaling pathway, negative regulation of interleukin-1 beta-mediated signaling pathway Definition: Any process that stops, prevents or reduces the frequency, rate or extent of interleukin-1-mediated signaling pathway.